{
  "term_id": "GO:0005634",
  "term_label": "nucleus",
  "gene_name": "Zinc finger protein basonuclin-1",
  "gene": "UniProtKB:Q01954",
  "gene_symbol": "BNC1"
}